vascular associated smooth muscle cell fate commitment [GO:0097081] (biological process) Definition: The commitment of cells to a vascular smooth muscle cell fate and their capacity to differentiate into vascular smooth muscle cells. A vascular smooth muscle cell is a non-striated, elongated, spindle-shaped cell found lining the blood vessels. Relationships: is a type of muscle cell fate commitment [GO:0042693]; is part of GO:0035886 Also known as: vascular smooth muscle cell fate commitment Subtypes: GO:0060949 Sources: GOC:BHF